{
  "gene_name": "Cadherin-1",
  "term_label": "calcium-dependent cell-cell adhesion",
  "gene": "UniProtKB:P12830",
  "gene_symbol": "CDH1",
  "term_id": "GO:0016339"
}